{
  "gene_name": "Protein FAM81B",
  "gene_symbol": "FAM81B",
  "term_label": "Unknown cellular component",
  "gene": "UniProtKB:Q96LP2",
  "term_id": "UNKNOWN:0003"
}